{
  "gene_name": "Synaptotagmin-2",
  "term_id": "GO:2000300",
  "term_label": "regulation of synaptic vesicle exocytosis",
  "gene": "UniProtKB:Q8N9I0",
  "gene_symbol": "SYT2"
}